{
  "term_id": "UNKNOWN:0002",
  "gene_name": "Olfactory receptor 4A16",
  "gene": "UniProtKB:Q8NH70",
  "gene_symbol": "OR4A16",
  "term_label": "Unknown biological process"
}